{
  "term_label": "membrane",
  "gene": "UniProtKB:Q92953",
  "term_id": "GO:0016020",
  "gene_name": "Potassium voltage-gated channel subfamily B member 2",
  "gene_symbol": "KCNB2"
}